{
  "term_id": "UNKNOWN:0003",
  "gene_name": "Corneodesmosin",
  "gene_symbol": "CDSN",
  "term_label": "Unknown cellular component",
  "gene": "UniProtKB:Q15517"
}